regulation of voltage-gated sodium channel activity [GO:1905150] (biological process) Definition: Any process that modulates the frequency, rate or extent of voltage-gated sodium channel activity. Also known as: regulation of voltage gated sodium channel activity, regulation of voltage-dependent sodium channel activity, regulation of voltage-gated sodium ion channel activity, regulation of voltage-sensitive sodium channel Subtypes: positive regulation of voltage-gated sodium channel activity [GO:1905152] Relationships: is a type of regulation of sodium ion transmembrane transporter activity [GO:2000649]; regulates voltage-gated sodium channel activity [GO:0005248] References: PMID:24198377 Sources: GOC:TermGenie, GO_REF:0000059